{
  "gene_symbol": "GAB4",
  "gene_name": "GRB2-associated-binding protein 4",
  "term_id": "GO:0005737",
  "term_label": "cytoplasm",
  "gene": "UniProtKB:Q2WGN9"
}